{
  "term_id": "GO:0016477",
  "gene_name": "Guanine nucleotide exchange factor VAV3",
  "term_label": "cell migration",
  "gene": "UniProtKB:Q9UKW4",
  "gene_symbol": "VAV3"
}